GABA-A receptor activity [GO:0004890] (molecular function) References: PMID:8974333 Relationships: is a type of GO:0016917 Also known as: ionotropic GABA receptor activity Regulation: regulated by regulation of GABA-A receptor activity [GO:0106040] Note: Note that this term represents an activity and not a gene product. Consider also annotating to the molecular function term 'chloride channel activity ; GO:0005254' and 'inhibitory extracellular ligand-gated ion channel activity ; GO:0005237'. Definition: Combining with the amino acid gamma-aminobutyric acid (GABA, 4-aminobutyrate) to initiate a change in cell activity. GABA-A receptors function as chloride channels.